regulation of timing of neuron differentiation [GO:0060164] (biological process) Sources: GOC:dph Relationships: is a type of regulation of neuron differentiation [GO:0045664]; is_a GO:0048505 Subtypes: GO:0060165 Definition: The process controlling the activation and/or rate at which a relatively unspecialized cell acquires features of a neuron.